{
  "gene_name": "Prolyl hydroxylase EGLN2",
  "gene": "UniProtKB:Q96KS0",
  "gene_symbol": "EGLN2",
  "term_label": "nucleus",
  "term_id": "GO:0005634"
}